{
  "gene_name": "Phosphatidylinositol N-acetylglucosaminyltransferase subunit Y",
  "term_id": "GO:0000506",
  "term_label": "glycosylphosphatidylinositol-N-acetylglucosaminyltransferase (GPI-GnT) complex",
  "gene_symbol": "PIGY",
  "gene": "UniProtKB:Q3MUY2"
}